negative regulation of mannan catabolic process [GO:2000995] (biological process) Sources: GOC:mengo_curators Relationships: is a type of negative regulation of cell wall polysaccharide catabolic process [GO:2000967]; is a type of regulation of mannan catabolic process [GO:2000994]; negatively regulates mannan catabolic process [GO:0046355] Definition: Any process that stops, prevents or reduces the frequency, rate or extent of mannan catabolic process. Also known as: negative regulation of mannan breakdown, negative regulation of mannan catabolism, negative regulation of mannan degradation